locomotion involved in locomotory behavior [GO:0031987] (biological process) Definition: Self-propelled movement of a cell or organism from one location to another in a behavioral context; the aspect of locomotory behavior having to do with movement. Subtypes: flight involved in flight behavior [GO:0060362] Sources: GOC:mah Relationships: is a type of locomotion [GO:0040011]; is part of locomotory behavior [GO:0007626] Regulation: regulated by regulation of locomotion involved in locomotory behavior [GO:0090325]; positively regulated by GO:0090326; negatively regulated by negative regulation of locomotion involved in locomotory behavior [GO:0090327] Also known as: locomotion during locomotory behaviour